{
  "gene_symbol": "GLA",
  "term_id": "GO:0016139",
  "gene_name": "Alpha-galactosidase A",
  "term_label": "glycoside catabolic process",
  "gene": "UniProtKB:P06280"
}